2,3-dihydro-2,3-dihydroxybenzoate dehydrogenase activity [GO:0008667] (molecular function) Definition: Catalysis of the reaction: (2S,3S)-2,3-dihydroxy-2,3-dihydrobenzoate + NAD+ = 2,3-dihydroxybenzoate + H+ + NADH. Sources: EC:1.3.1.28, RHEA:23824 Also known as: 2,3-DHB dehydrogenase activity, 2,3-dihydro-2,3-dihydroxybenzoate:NAD+ oxidoreductase activity Relationships: is a type of oxidoreductase activity, acting on the CH-CH group of donors, NAD or NADP as acceptor [GO:0016628]